{
  "term_id": "GO:0005615",
  "gene": "UniProtKB:Q99102",
  "term_label": "extracellular space",
  "gene_name": "Mucin-4",
  "gene_symbol": "MUC4"
}